adaptation of signaling pathway by response to pheromone involved in conjugation with cellular fusion [GO:0000754] (biological process) Definition: In organisms that undergo conjugation with cellular fusion, the process resulting in desensitization following exposure to pheromone stimulus that act to down-regulate further stimulation or block initial conjugation responses. An example of this is the adaptation to pheromone during conjugation with cellular fusion in Saccharomyces cerevisiae. Sources: GOC:clt Also known as: adaptation of signalling pathway by response to pheromone involved in conjugation with cellular fusion, desensitization to pheromone during conjugation with cellular fusion, adaptation to pheromone during conjugation with cellular fusion Relationships: is a type of adaptation of signaling pathway [GO:0023058]; is part of response to pheromone triggering conjugation with cellular fusion [GO:0000749] Subtypes: re-entry into mitotic cell cycle after pheromone arrest [GO:0000321]